radial spoke 1 [GO:0120333] (cellular component) References: PMID:22754630 Sources: GOC:krc Relationships: is a type of radial spoke [GO:0001534] Definition: The radial spoke of each group of radial spokes, whether grouped as triplets or doublets, that is most proximal to the base of the cilium. Radial spoke 1 (RS1), similarly to radial spoke 2, is comprised of four domains: 1) a very short base anchored to the A microtubule, 2) an elongaged stalk, 3) a bifurcated neck, and 4) an orthogonal head. The base of RS1 is connected to the tail of the inner dynein arm a/d. Also known as: RS1